{
  "term_id": "GO:0005525",
  "gene_symbol": "RABL6",
  "gene_name": "Rab-like protein 6",
  "term_label": "GTP binding",
  "gene": "UniProtKB:Q3YEC7"
}